{
  "gene_name": "Uncharacterized protein SPEM3",
  "term_label": "flagellated sperm motility",
  "gene": "UniProtKB:A0A1B0GUW6",
  "gene_symbol": "SPEM3",
  "term_id": "GO:0030317"
}